central nervous system segmentation [GO:0035283] (biological process) Definition: Division of the central nervous system into a series of semi-repetitive parts or segments. Relationships: is a type of GO:0035282; is part of central nervous system development [GO:0007417] Sources: GOC:bf